{
  "gene": "UniProtKB:Q8N5H3",
  "term_label": "negative regulation of SMAD protein signal transduction",
  "gene_name": "Leucine repeat adapter protein 25",
  "term_id": "GO:0060392",
  "gene_symbol": "FAM89B"
}